{
  "gene_symbol": "PIEZO1",
  "gene": "UniProtKB:Q92508",
  "term_label": "plasma membrane",
  "term_id": "GO:0005886",
  "gene_name": "Piezo-type mechanosensitive ion channel component 1"
}